{
  "gene": "UniProtKB:O76027",
  "gene_name": "Annexin A9",
  "term_id": "GO:0001786",
  "term_label": "phosphatidylserine binding",
  "gene_symbol": "ANXA9"
}